{
  "gene_symbol": "TMEM14C",
  "gene_name": "Transmembrane protein 14C",
  "term_label": "heme biosynthetic process",
  "term_id": "GO:0006783",
  "gene": "UniProtKB:Q9P0S9"
}